{
  "gene": "UniProtKB:Q9HC07",
  "term_id": "GO:0005384",
  "gene_name": "Transmembrane protein 165",
  "gene_symbol": "TMEM165",
  "term_label": "manganese ion transmembrane transporter activity"
}